rhodopsin catabolic process [GO:0046155] (biological process) Definition: The chemical reactions and pathways resulting in the breakdown of rhodopsin, a brilliant purplish-red, light-sensitive visual pigment found in the rod cells of the retinas. Sources: ISBN:0198506732 Also known as: rhodopsin breakdown, rhodopsin catabolism, rhodopsin degradation Relationships: is_a xanthophyll catabolic process [GO:0016124]; is a type of protein catabolic process [GO:0030163]; is a type of eye pigment catabolic process [GO:0046151]; is_a GO:0046164; is a type of GO:1902644